{
  "term_id": "UNKNOWN:0002",
  "gene_name": "Serine_threonine-protein kinase PRP4 homolog",
  "gene": "UniProtKB:Q13523",
  "term_label": "Unknown biological process",
  "gene_symbol": "PRPF4B"
}